{
  "gene_symbol": "SDHD",
  "gene": "UniProtKB:O14521",
  "term_id": "GO:0045273",
  "gene_name": "Succinate dehydrogenase [ubiquinone] cytochrome b small subunit, mitochondrial",
  "term_label": "respiratory chain complex II (succinate dehydrogenase)"
}